{
  "gene_symbol": "DNTTIP1",
  "gene": "UniProtKB:Q9H147",
  "term_id": "GO:0005634",
  "term_label": "nucleus",
  "gene_name": "Deoxynucleotidyltransferase terminal-interacting protein 1"
}